{
  "gene_symbol": "NIM1K",
  "term_label": "Unknown cellular component",
  "term_id": "UNKNOWN:0003",
  "gene_name": "Serine_threonine-protein kinase NIM1",
  "gene": "UniProtKB:Q8IY84"
}